{
  "gene_symbol": "SOX18",
  "term_label": "lymphangiogenesis",
  "gene": "UniProtKB:P35713",
  "gene_name": "Transcription factor SOX-18",
  "term_id": "GO:0001946"
}